{
  "gene_name": "Claudin-8",
  "term_id": "GO:0160184",
  "gene_symbol": "CLDN8",
  "term_label": "paracellular transport",
  "gene": "UniProtKB:P56748"
}